{
  "term_id": "GO:0003924",
  "gene_name": "Neuronal-specific septin-3",
  "gene_symbol": "SEPTIN3",
  "term_label": "GTPase activity",
  "gene": "UniProtKB:Q9UH03"
}